{
  "gene": "UniProtKB:Q6PEY0",
  "term_label": "cell-cell signaling",
  "term_id": "GO:0007267",
  "gene_name": "Gap junction beta-7 protein",
  "gene_symbol": "GJB7"
}